{
  "gene": "UniProtKB:Q8N3U4",
  "gene_symbol": "STAG2",
  "term_id": "GO:0003682",
  "gene_name": "Cohesin subunit SA-2",
  "term_label": "chromatin binding"
}